establishment or maintenance of apical/basal cell polarity [GO:0035088] (biological process) Subtypes: establishment of apical/basal cell polarity [GO:0035089], maintenance of apical/basal cell polarity [GO:0035090], establishment or maintenance of epithelial cell apical/basal polarity [GO:0045197] Definition: Any cellular process that results in the specification, formation or maintenance polarization of a cell's architecture along its apical/basal axis so that the apical and basal regions of the cell have different membrane, extracellular matrix and sub-membrane cellular components. References: PMID:10934483 Sources: GOC:bf, GOC:mah Relationships: is a type of establishment or maintenance of bipolar cell polarity [GO:0061245]